{
  "gene_name": "Nephrocystin-1",
  "term_label": "cytoplasm",
  "term_id": "GO:0005737",
  "gene": "UniProtKB:O15259",
  "gene_symbol": "NPHP1"
}